{
  "term_label": "neurotransmitter receptor activity",
  "term_id": "GO:0030594",
  "gene_symbol": "HTR5A",
  "gene_name": "5-hydroxytryptamine receptor 5A",
  "gene": "UniProtKB:P47898"
}